{
  "term_id": "GO:0008574",
  "gene": "UniProtKB:O60282",
  "gene_symbol": "KIF5C",
  "gene_name": "Kinesin heavy chain isoform 5C",
  "term_label": "plus-end-directed microtubule motor activity"
}